lipid sensor activity [GO:0106254] (molecular function) Definition: Binding to and responding, e.g. by conformational change, to changes in the cellular level of a lipid. References: PMID:30075144 Sources: GOC:vw Also known as: lipid sensing activity Relationships: is a type of molecular sensor activity [GO:0140299] Subtypes: sterol sensor activity [GO:0032935], phosphatidylinositol-4,5-bisphosphate sensor activity [GO:0140550]